{
  "term_label": "small GTPase binding",
  "term_id": "GO:0031267",
  "gene_symbol": "RIN1",
  "gene_name": "Ras and Rab interactor 1",
  "gene": "UniProtKB:Q13671"
}